megasporogenesis [GO:0009554] (BP) Definition: The process in which the megasporocyte undergoes meiosis, giving rise to four haploid megaspores in the nucellus. Sources: GOC:mtg_plant, GOC:tb Also known as: megaspore development, megaspore mother cell meiosis, meiosis of the megasporocyte, meiotic division of the megasporocyte Relationships: is a type of plant-type sporogenesis [GO:0048236]; is part of GO:0009553